{
  "gene_name": "Gephyrin",
  "term_label": "postsynaptic membrane",
  "gene_symbol": "GPHN",
  "term_id": "GO:0045211",
  "gene": "UniProtKB:Q9NQX3"
}